{
  "gene_name": "UDP-glucuronosyltransferase 1-6",
  "gene": "UniProtKB:P19224",
  "term_id": "GO:0008194",
  "term_label": "UDP-glycosyltransferase activity",
  "gene_symbol": "UGT1A6"
}